pentose-phosphate shunt [GO:0006098] (biological process) Relationships: is a type of GO:0006740; is a type of glucose 6-phosphate metabolic process [GO:0051156]; has part GO:0009051; has part pentose-phosphate shunt, non-oxidative branch [GO:0009052] Regulation: regulated by GO:0043456; negatively regulated by negative regulation of pentose-phosphate shunt [GO:1905856]; positively regulated by positive regulation of pentose-phosphate shunt [GO:1905857] Also known as: hexose monophosphate pathway, pentose phosphate pathway, pentose phosphate shunt, pentose-phosphate pathway Definition: The metabolic process in which glucose-6-phosphate is oxidized to form carbon dioxide (CO2) and ribulose 5-phosphate, coupled to reduction of NADP+ to NADPH; ribulose 5-P then enters a series of reactions that can yield biosynthetic precursors (ribose-5-phosphate and erythrose-4-phosphate) and glycolytic intermediates (fructose-6-phosphate and glyceraldehyde-3-phosphate). Sources: GOC:pde, ISBN:0198506732, MetaCyc:PENTOSE-P-PWY